phosphomevalonate kinase activity [GO:0004631] (molecular function) Sources: EC:2.7.4.2, RHEA:16341 Relationships: is a type of kinase activity [GO:0016301]; is_a phosphotransferase activity, phosphate group as acceptor [GO:0016776] Definition: Catalysis of the reaction: (R)-5-phosphomevalonate + ATP = (R)-5-diphosphomevalonate + ADP + H+. Also known as: 5-phosphomevalonate kinase activity, ATP:(R)-5-phosphomevalonate phosphotransferase activity, ATP:5-phosphomevalonate phosphotransferase activity, mevalonate phosphate kinase activity, mevalonate-5-phosphate kinase activity, mevalonic acid phosphate kinase activity